{
  "term_id": "GO:0016712",
  "term_label": "oxidoreductase activity, acting on paired donors, with incorporation or reduction of molecular oxygen, reduced flavin or flavoprotein as one donor, and incorporation of one atom of oxygen",
  "gene": "UniProtKB:P20813",
  "gene_name": "Cytochrome P450 2B6",
  "gene_symbol": "CYP2B6"
}